{
  "gene_symbol": "CCP110",
  "gene": "UniProtKB:O43303",
  "term_id": "GO:0007099",
  "gene_name": "Centriolar coiled-coil protein of 110 kDa",
  "term_label": "centriole replication"
}